positive regulation of amyloid precursor protein catabolic process [GO:1902993] (biological process) Relationships: is a type of GO:0051247; is a type of regulation of amyloid precursor protein catabolic process [GO:1902991]; positively regulates amyloid precursor protein catabolic process [GO:0042987] Also known as: positive regulation of APP catabolic process, positive regulation of APP catabolism, positive regulation of amyloid precursor protein breakdown, positive regulation of amyloid precursor protein catabolism, positive regulation of amyloid precursor protein degradation, up regulation of APP catabolic process, up regulation of APP catabolism, up regulation of amyloid precursor protein breakdown, up regulation of amyloid precursor protein catabolic process, up regulation of amyloid precursor protein catabolism, up regulation of amyloid precursor protein degradation, up-regulation of APP catabolic process, up-regulation of APP catabolism, up-regulation of amyloid precursor protein breakdown, up-regulation of amyloid precursor protein catabolic process, up-regulation of amyloid precursor protein catabolism, up-regulation of amyloid precursor protein degradation, upregulation of APP catabolic process, upregulation of APP catabolism, upregulation of amyloid precursor protein breakdown, upregulation of amyloid precursor protein catabolic process, upregulation of amyloid precursor protein catabolism, upregulation of amyloid precursor protein degradation, activation of APP catabolic process, activation of APP catabolism, activation of amyloid precursor protein breakdown, activation of amyloid precursor protein catabolic process, activation of amyloid precursor protein catabolism, activation of amyloid precursor protein degradation References: PMID:24499793 Sources: GOC:PARL, GOC:TermGenie, GOC:rl, GO_REF:0000058 Definition: Any process that activates or increases the frequency, rate or extent of amyloid precursor protein catabolic process. Subtypes: positive regulation of amyloid-beta formation [GO:1902004]